{
  "gene": "UniProtKB:Q96R54",
  "term_id": "GO:0005549",
  "gene_name": "Olfactory receptor 14A2",
  "gene_symbol": "OR14A2",
  "term_label": "odorant binding"
}